innate immune receptor activity [GO:0140376] (molecular function) Relationships: is_a immune receptor activity [GO:0140375] Definition: Receiving a signal and transmitting it in a cell to initiate an innate immune response. References: PMID:28921463, PMID:31415752